{
  "term_id": "GO:0050766",
  "gene_symbol": "MBL2",
  "gene_name": "Mannose-binding protein C",
  "term_label": "positive regulation of phagocytosis",
  "gene": "UniProtKB:P11226"
}